{
  "term_id": "GO:0005856",
  "gene_symbol": "SPRY2",
  "term_label": "cytoskeleton",
  "gene": "UniProtKB:O43597",
  "gene_name": "Protein sprouty homolog 2"
}